{
  "gene_name": "ELMO domain-containing protein 3",
  "term_label": "cilium assembly",
  "gene_symbol": "ELMOD3",
  "gene": "UniProtKB:Q96FG2",
  "term_id": "GO:0060271"
}